{
  "gene_symbol": "GRIA3",
  "term_id": "GO:0050804",
  "term_label": "modulation of chemical synaptic transmission",
  "gene": "UniProtKB:P42263",
  "gene_name": "Glutamate receptor 3"
}